{
  "gene": "UniProtKB:Q9NY47",
  "term_label": "Unknown biological process",
  "gene_symbol": "CACNA2D2",
  "gene_name": "Voltage-dependent calcium channel subunit alpha-2_delta-2",
  "term_id": "UNKNOWN:0002"
}